{
  "term_label": "ubiquitin binding",
  "term_id": "GO:0043130",
  "gene": "UniProtKB:Q99816",
  "gene_symbol": "TSG101",
  "gene_name": "Tumor susceptibility gene 101 protein"
}